{
  "gene_name": "Putative uncharacterized protein encoded by LINC01555",
  "gene": "UniProtKB:Q8NAE3",
  "gene_symbol": "LINC01555",
  "term_label": "Unknown biological process",
  "term_id": "UNKNOWN:0002"
}